{
  "gene_name": "Mitogen-activated protein kinase 13",
  "gene_symbol": "MAPK13",
  "gene": "UniProtKB:O15264",
  "term_id": "GO:0035556",
  "term_label": "intracellular signal transduction"
}